{
  "term_label": "nuclear-transcribed mRNA catabolic process",
  "gene_name": "Superkiller complex protein 3",
  "gene": "UniProtKB:Q6PGP7",
  "gene_symbol": "SKIC3",
  "term_id": "GO:0000956"
}